mitochondrial protein processing [GO:0034982] (biological process) Relationships: is a type of GO:0016485; occurs in mitochondrion [GO:0005739] Also known as: mitochondrial protein modification Sources: GOC:curators Subtypes: protein processing involved in protein targeting to mitochondrion [GO:0006627] Definition: The peptide cleavage of mitochondrial proteins, including cleavage contributing to their import.